Glc3Man9GlcNAc2 oligosaccharide glucosidase activity [GO:0004573] (molecular function) Definition: Catalysis of the exohydrolysis of the non-reducing terminal glucose residue in the mannosyl-oligosaccharide Glc(3)Man(9)GlcNAc(2). Sources: EC:3.2.1.106 Also known as: mannosyl-oligosaccharide glucosidase (processing A-glucosidase I) activity, trimming glucosidase I, mannosyl-oligosaccharide glucohydrolase activity, mannosyl-oligosaccharide glucosidase activity, processing A-glucosidase I activity Relationships: is a type of GO:0090599